{
  "gene_symbol": "ACOD1",
  "gene": "UniProtKB:A6NK06",
  "term_id": "GO:0002760",
  "gene_name": "Cis-aconitate decarboxylase",
  "term_label": "positive regulation of antimicrobial humoral response"
}